{
  "term_id": "GO:0015813",
  "gene_symbol": "SLC25A22",
  "gene": "UniProtKB:Q9H936",
  "term_label": "L-glutamate transmembrane transport",
  "gene_name": "Mitochondrial glutamate carrier 1"
}